{
  "term_label": "heterophilic cell-cell adhesion",
  "gene": "UniProtKB:A1L1A6",
  "gene_name": "Immunoglobulin superfamily member 23",
  "gene_symbol": "IGSF23",
  "term_id": "GO:0007157"
}